{
  "term_id": "UNKNOWN:0003",
  "term_label": "Unknown cellular component",
  "gene": "UniProtKB:Q5SWX8",
  "gene_name": "Protein odr-4 homolog",
  "gene_symbol": "ODR4"
}